phospholipase C-activating angiotensin-activated signaling pathway involved in heart process [GO:0086099] (biological process) References: PMID:17376402 Sources: GOC:BHF, GOC:mtg_cardiac_conduct_nov11 Definition: An angiotensin-mediated signaling pathway that contributes to a circulatory system process carried out by the heart, where the activated receptor transmits the signal via Gq-mediated activation of phospholipase C (PLC). PLC hydrolyses phosphatidylinositol 4,5-bisphosphate (PIP2) into the second messengers inositol-1,4,5,-triphosphate (IP3) and diacylglycerol (DAG). DAG activates protein kinase C (PKC), whilst IP3 binds intracellular receptors to induce the release of Ca2+ from intracellular stores. Relationships: is a type of phospholipase C-activating angiotensin-activated signaling pathway [GO:0086097]; is_a angiotensin-activated signaling pathway involved in heart process [GO:0086098] Also known as: Gq-coupled angiotensin receptor signaling pathway involved in heart process, PLC-activating angiotensin receptor signaling pathway involved in heart process, angiotensin receptor signaling pathway via activation of phospholipase C involved in heart process, cardiac angiotensin receptor signaling pathway via activation of PLC, phospholipase C-activating angiotensin-mediated signaling pathway involved in heart process